{
  "gene_symbol": "ANAPC5",
  "gene_name": "Anaphase-promoting complex subunit 5",
  "gene": "UniProtKB:Q9UJX4",
  "term_id": "GO:0070979",
  "term_label": "protein K11-linked ubiquitination"
}